{
  "gene_name": "Protein SFI1 homolog",
  "term_id": "UNKNOWN:0003",
  "gene": "UniProtKB:A8K8P3",
  "gene_symbol": "SFI1",
  "term_label": "Unknown cellular component"
}